{
  "term_label": "actin filament organization",
  "gene": "UniProtKB:P09493",
  "gene_symbol": "TPM1",
  "gene_name": "Tropomyosin alpha-1 chain",
  "term_id": "GO:0007015"
}